{
  "gene": "UniProtKB:Q8N6D2",
  "gene_symbol": "RNF182",
  "gene_name": "E3 ubiquitin-protein ligase RNF182",
  "term_label": "ubiquitin-protein transferase activity",
  "term_id": "GO:0004842"
}